{
  "term_id": "GO:0005634",
  "gene_symbol": "PTP4A1",
  "gene": "UniProtKB:Q93096",
  "gene_name": "Protein tyrosine phosphatase type IVA 1",
  "term_label": "nucleus"
}